{
  "term_label": "cytosol",
  "gene": "UniProtKB:Q9UMX0",
  "gene_name": "Ubiquilin-1",
  "term_id": "GO:0005829",
  "gene_symbol": "UBQLN1"
}